{
  "term_id": "GO:0000124",
  "gene_symbol": "SGF29",
  "gene": "UniProtKB:Q96ES7",
  "term_label": "SAGA complex",
  "gene_name": "SAGA-associated factor 29"
}